{
  "term_id": "GO:0015179",
  "gene": "UniProtKB:Q08AI6",
  "term_label": "L-amino acid transmembrane transporter activity",
  "gene_symbol": "SLC38A11",
  "gene_name": "Putative sodium-coupled neutral amino acid transporter 11"
}